positive regulation of mesenchymal cell proliferation involved in ureter development [GO:2000729] (biological process) Also known as: positive regulation of ureter mesenchymal cell proliferation, positive regulation of ureteral mesenchymal cell proliferation Definition: Any process that activates or increases the frequency, rate or extent of mesenchymal cell proliferation involved in ureter development. Relationships: is a type of positive regulation of mesenchymal cell proliferation [GO:0002053]; is a type of positive regulation of developmental process [GO:0051094]; is a type of regulation of mesenchymal cell proliferation involved in ureter development [GO:0072199]; positively regulates mesenchymal cell proliferation involved in ureter development [GO:0072198] Sources: GOC:obol